crystalloid [GO:0044312] (cellular component) Relationships: is a type of intracellular membraneless organelle [GO:0043232]; is part of cytoplasm [GO:0005737] Definition: A transient, cytoplasmic organelle found in Plasmodium species that resembles a cytoplasmic inclusion body and whose function is poorly understood. Crystalloids form in ookinetes and disappear after ookinete-to-oocyst transformation. References: PMID:19932717 Sources: GOC:jl